response to erythromycin [GO:1901323] (biological process) Subtypes: cellular response to erythromycin [GO:0072743] Sources: GOC:TermGenie Relationships: is a type of GO:1901700 Definition: Any process that results in a change in state or activity of a cell or an organism (in terms of movement, secretion, enzyme production, gene expression, etc.) as a result of an erythromycin stimulus.